{
  "gene_name": "Tripartite motif-containing protein 49",
  "term_id": "GO:0010468",
  "term_label": "regulation of gene expression",
  "gene": "UniProtKB:P0CI25",
  "gene_symbol": "TRIM49"
}